{
  "term_label": "extracellular space",
  "gene_name": "P-selectin",
  "term_id": "GO:0005615",
  "gene_symbol": "SELP",
  "gene": "UniProtKB:P16109"
}